{
  "term_label": "glutathione peroxidase activity",
  "gene_symbol": "GPX6",
  "gene_name": "Glutathione peroxidase 6",
  "term_id": "GO:0004602",
  "gene": "UniProtKB:P59796"
}